{
  "gene_name": "Defensin-6",
  "term_label": "extracellular space",
  "term_id": "GO:0005615",
  "gene": "UniProtKB:Q01524",
  "gene_symbol": "DEFA6"
}